aminoglycan biosynthetic process [GO:0006023] (biological process) Subtypes: glycosaminoglycan biosynthetic process [GO:0006024], chitin biosynthetic process [GO:0006031], GO:0030311 Relationships: is a type of aminoglycan metabolic process [GO:0006022]; is a type of macromolecule biosynthetic process [GO:0009059]; is a type of carbohydrate derivative biosynthetic process [GO:1901137] Also known as: aminoglycan anabolism, aminoglycan biosynthesis, aminoglycan formation, aminoglycan synthesis Definition: The chemical reactions and pathways resulting in the formation of aminoglycans, any polymer containing amino groups that consists of more than about 10 monosaccharide residues joined to each other by glycosidic linkages. Sources: GOC:ai, ISBN:0198506732